{
  "term_id": "GO:0005881",
  "term_label": "cytoplasmic microtubule",
  "gene": "UniProtKB:Q9P2G4",
  "gene_name": "Microtubule-associated protein 10",
  "gene_symbol": "MAP10"
}